translation repressor complex [GO:1903502] (cellular component) Note: An example of this is Eif4e in drome (P48598) in PMID:14723848 (inferred from physical interaction). Definition: A protein complex which is capable of translation repressor activity. Subtypes: eif4e-cup complex [GO:1990500] References: PMID:14723848 Sources: GOC:TermGenie, GOC:bhm, GO_REF:0000088 Relationships: is a type of protein-containing complex [GO:0032991]